protein localization to actomyosin contractile ring [GO:1990179] (biological process) Subtypes: protein localization to mitotic actomyosin contractile ring [GO:1904498] Relationships: is a type of protein localization to cell cortex [GO:0072697]; is_a protein localization to cell division site [GO:0072741]; is a type of protein localization to actin cytoskeleton [GO:1903119] Also known as: protein localisation to actomyosin contractile ring Definition: A process in which a protein is transported to, or maintained at, the actomyosin contractile ring. References: PMID:23349808 Sources: GOC:mah